regulation of estrogen biosynthetic process [GO:1904076] (biological process) Relationships: is_a regulation of hormone biosynthetic process [GO:0046885]; is a type of regulation of steroid biosynthetic process [GO:0050810]; regulates estrogen biosynthetic process [GO:0006703] Subtypes: GO:1904077, GO:1904078 Also known as: regulation of estrogen anabolism, regulation of estrogen biosynthesis, regulation of estrogen formation, regulation of estrogen synthesis, regulation of oestrogen biosynthesis, regulation of oestrogen biosynthetic process Definition: Any process that modulates the frequency, rate or extent of estrogen biosynthetic process. References: PMID:24530842 Sources: GOC:TermGenie, GO_REF:0000058